{
  "gene": "UniProtKB:Q8NEJ0",
  "term_id": "UNKNOWN:0002",
  "gene_name": "Dual specificity protein phosphatase 18",
  "gene_symbol": "DUSP18",
  "term_label": "Unknown biological process"
}